negative regulation of transcription from RNA polymerase II promoter by glucose [GO:0061987] (biological process) Relationships: is a type of regulation of transcription from RNA polymerase II promoter by glucose [GO:0000430]; is a type of negative regulation of transcription by glucose [GO:0061986] References: PMID:11875061 Subtypes: GO:0000433 Definition: Any process involving glucose that decreases the frequency, rate or extent or transcription from an RNA polymerase II promoter.